{
  "gene_name": "Protein TOPAZ1",
  "gene_symbol": "TOPAZ1",
  "term_label": "Unknown cellular component",
  "gene": "UniProtKB:Q8N9V7",
  "term_id": "UNKNOWN:0003"
}